protein phosphatase 4 complex [GO:0030289] (cellular component) Definition: A protein serine/threonine phosphatase complex formed by the catalytic subunit of protein phosphatase 4 plus one or more regulatory subunits. References: PMID:10026142 Sources: GOC:bhm Relationships: is_a protein serine/threonine phosphatase complex [GO:0008287]